{
  "term_label": "perinuclear region of cytoplasm",
  "gene_symbol": "EHD2",
  "gene": "UniProtKB:Q9NZN4",
  "gene_name": "EH domain-containing protein 2",
  "term_id": "GO:0048471"
}